{
  "gene_name": "Exosome component 10",
  "gene_symbol": "EXOSC10",
  "gene": "UniProtKB:Q01780",
  "term_label": "3'-5'-RNA exonuclease activity",
  "term_id": "GO:0000175"
}